{
  "gene": "UniProtKB:Q8WVS4",
  "gene_name": "Cytoplasmic dynein 2 intermediate chain 1",
  "gene_symbol": "DYNC2I1",
  "term_id": "GO:0000242",
  "term_label": "pericentriolar material"
}